mammary gland bud formation [GO:0060615] (biological process) Relationships: is a type of morphogenesis of embryonic epithelium [GO:0016331]; is a type of anatomical structure formation involved in morphogenesis [GO:0048646]; is part of mammary gland bud morphogenesis [GO:0060648] References: PMID:12558599 Sources: GOC:dph Definition: The morphogenetic process in which a bud forms from the mammary placode. A mammary bud is bulb of epithelial cells that is distinct from the surrounding epidermis.